{
  "gene_symbol": "MPHOSPH10",
  "term_id": "UNKNOWN:0001",
  "gene_name": "U3 small nucleolar ribonucleoprotein protein MPP10",
  "term_label": "Unknown molecular function",
  "gene": "UniProtKB:O00566"
}